{
  "gene_symbol": "OR10Q1",
  "gene_name": "Olfactory receptor 10Q1",
  "term_label": "Unknown biological process",
  "gene": "UniProtKB:Q8NGQ4",
  "term_id": "UNKNOWN:0002"
}